{
  "term_label": "Unknown molecular function",
  "gene_name": "Immunoglobulin heavy diversity 3-3 (Fragment)",
  "term_id": "UNKNOWN:0001",
  "gene_symbol": "IGHD3-3",
  "gene": "UniProtKB:A0A0J9YWD0"
}